{
  "gene_symbol": "UNC93A",
  "term_id": "UNKNOWN:0003",
  "term_label": "Unknown cellular component",
  "gene": "UniProtKB:Q86WB7",
  "gene_name": "Protein unc-93 homolog A"
}